regulation of c-di-GMP signaling [GO:0061940] (biological process) Relationships: is a type of regulation of cell communication [GO:0010646]; is a type of GO:0023051; regulates GO:0061939 References: PMID:22864416 Definition: Any process that modulates the rate frequency or extent of c-di-GMP signaling. Subtypes: positive regulation of c-di-GMP signaling [GO:0061941], negative regulation of c-di-GMP signaling [GO:0061942]